{
  "gene": "UniProtKB:Q9Y5J3",
  "gene_symbol": "HEY1",
  "term_label": "circulatory system development",
  "term_id": "GO:0072359",
  "gene_name": "Hairy_enhancer-of-split related with YRPW motif protein 1"
}